negative regulation of hepatic stellate cell proliferation [GO:1904898] (biological process) References: PMID:15358192 Sources: GOC:TermGenie, GO_REF:0000058 Relationships: is a type of negative regulation of fibroblast proliferation [GO:0048147]; is a type of regulation of hepatic stellate cell proliferation [GO:1904897]; negatively regulates hepatic stellate cell proliferation [GO:1990922] Also known as: down regulation of Ito cell proliferation, down regulation of hepatic perisinusoidal cell proliferation, down regulation of hepatic stellate cell proliferation, down regulation of perisinusoidal cell proliferation, down-regulation of Ito cell proliferation, down-regulation of hepatic perisinusoidal cell proliferation, down-regulation of hepatic stellate cell proliferation, down-regulation of perisinusoidal cell proliferation, downregulation of Ito cell proliferation, downregulation of hepatic perisinusoidal cell proliferation, downregulation of hepatic stellate cell proliferation, downregulation of perisinusoidal cell proliferation, negative regulation of Ito cell proliferation, negative regulation of hepatic perisinusoidal cell proliferation, negative regulation of perisinusoidal cell proliferation, inhibition of Ito cell proliferation, inhibition of hepatic perisinusoidal cell proliferation, inhibition of hepatic stellate cell proliferation, inhibition of perisinusoidal cell proliferation Definition: Any process that stops, prevents or reduces the frequency, rate or extent of hepatic stellate cell proliferation.